{
  "term_id": "GO:0016020",
  "gene_symbol": "POTEKP",
  "gene": "UniProtKB:Q9BYX7",
  "gene_name": "Putative beta-actin-like protein 3",
  "term_label": "membrane"
}